{
  "gene_name": "Blood vessel epicardial substance",
  "term_id": "GO:0030552",
  "term_label": "cAMP binding",
  "gene_symbol": "BVES",
  "gene": "UniProtKB:Q8NE79"
}